{
  "gene": "UniProtKB:A0A455ZAR2",
  "gene_symbol": "LINC-PINT",
  "term_id": "UNKNOWN:0002",
  "term_label": "Unknown biological process",
  "gene_name": "Transcriptional regulator PINT87aa"
}